funalenone biosynthetic process [GO:1901366] (biological process) Definition: The chemical reactions and pathways resulting in the formation of funalenone. Also known as: funalenone anabolism, funalenone biosynthesis, funalenone formation, funalenone synthesis Relationships: is a type of ketone biosynthetic process [GO:0042181]; is a type of phenol-containing compound biosynthetic process [GO:0046189]; is a type of olefinic compound biosynthetic process [GO:0120255] Sources: GOC:TermGenie, GOC:di